{
  "term_id": "GO:0060070",
  "gene": "UniProtKB:Q8N474",
  "gene_name": "Secreted frizzled-related protein 1",
  "term_label": "canonical Wnt signaling pathway",
  "gene_symbol": "SFRP1"
}